{
  "gene_name": "Ankyrin repeat domain-containing protein 11",
  "gene": "UniProtKB:Q6UB99",
  "term_label": "Unknown molecular function",
  "gene_symbol": "ANKRD11",
  "term_id": "UNKNOWN:0001"
}